cellular response to potassium ion [GO:0035865] (biological process) Also known as: cellular response to K+ ion, cellular response to potassium Definition: Any process that results in a change in state or activity of a cell (in terms of movement, secretion, enzyme production, gene expression, etc.) as a result of a potassium ion stimulus. Sources: GOC:yaf Relationships: is a type of response to potassium ion [GO:0035864]; is a type of cellular response to metal ion [GO:0071248]